{
  "term_label": "cell development",
  "gene": "UniProtKB:O15169",
  "term_id": "GO:0048468",
  "gene_symbol": "AXIN1",
  "gene_name": "Axin-1"
}